ubiquitin-dependent protein catabolic process via the C-end degron rule pathway [GO:0140627] (biological process) Also known as: DesCEND Definition: The chemical reactions and pathways resulting in the breakdown of a protein or peptide covalently tagged with ubiquitin, via the DesCEND (destruction via C-end degron) pathway. In the DesCEND pathway, C-terminal residues (C-end degrons) in substrates are recognized by Cul2-RING and Cul4-RING E3 ligases, whereupon the substrates are linked to ubiquitin and then delivered to the proteasome for degradation. C-end degrons can be present in full-length proteins, truncated proteins or proteolytically cleaved forms. Relationships: is a type of proteasome-mediated ubiquitin-dependent protein catabolic process [GO:0043161] References: PMID:29775578, PMID:29779948